{
  "term_id": "GO:0030425",
  "gene_symbol": "CNIH3",
  "gene": "UniProtKB:Q8TBE1",
  "gene_name": "Protein cornichon homolog 3",
  "term_label": "dendrite"
}